{
  "gene": "UniProtKB:Q9Y3Y4",
  "gene_symbol": "PYGO1",
  "gene_name": "Pygopus homolog 1",
  "term_id": "GO:0001822",
  "term_label": "kidney development"
}